{
  "gene_symbol": "EPPIN",
  "gene_name": "Eppin",
  "term_id": "GO:1901318",
  "gene": "UniProtKB:O95925",
  "term_label": "negative regulation of flagellated sperm motility"
}